{
  "gene_name": "MAGUK p55 subfamily member 7",
  "gene_symbol": "MPP7",
  "term_id": "GO:0005911",
  "term_label": "cell-cell junction",
  "gene": "UniProtKB:Q5T2T1"
}